{
  "gene_symbol": "CTSH",
  "term_id": "GO:0005764",
  "gene_name": "Pro-cathepsin H",
  "gene": "UniProtKB:P09668",
  "term_label": "lysosome"
}